{
  "term_label": "cytoplasm",
  "gene": "UniProtKB:Q7Z6Z6",
  "gene_symbol": "PNPLA5",
  "gene_name": "Patatin-like phospholipase domain-containing protein 5",
  "term_id": "GO:0005737"
}